{
  "gene_symbol": "STMN3",
  "term_label": "tubulin binding",
  "gene": "UniProtKB:Q9NZ72",
  "gene_name": "Stathmin-3",
  "term_id": "GO:0015631"
}